sphingoid biosynthetic process [GO:0046520] (biological process) Also known as: sphingoid anabolism, sphingoid biosynthesis, sphingoid formation, sphingoid synthesis Subtypes: sphinganine biosynthetic process [GO:0046511], sphingosine biosynthetic process [GO:0046512], phytosphingosine biosynthetic process [GO:0071602] Sources: ISBN:0198506732 Relationships: is a type of sphingolipid biosynthetic process [GO:0030148]; is a type of GO:0046519 Definition: The chemical reactions and pathways resulting in the formation of sphingoids, any of a class of compounds comprising sphinganine and its homologues and stereoisomers, and derivatives of these compounds.